positive regulation of cardiac neural crest cell migration involved in outflow tract morphogenesis [GO:1905312] (BP) Definition: Any process that activates or increases the frequency, rate or extent of cardiac neural crest cell migration involved in outflow tract morphogenesis. References: PMID:17628518 Sources: GOC:BHF, GOC:TermGenie, GOC:rl, GO_REF:0000058 Relationships: is a type of positive regulation of cell migration [GO:0030335]; is a type of regulation of cardiac neural crest cell migration involved in outflow tract morphogenesis [GO:1905310]; positively regulates cardiac neural crest cell migration involved in outflow tract morphogenesis [GO:0003253] Also known as: up regulation of cardiac neural crest cell migration involved in outflow tract morphogenesis, up-regulation of cardiac neural crest cell migration involved in outflow tract morphogenesis, upregulation of cardiac neural crest cell migration involved in outflow tract morphogenesis, activation of cardiac neural crest cell migration involved in outflow tract morphogenesis